{
  "gene_name": "Centrosomal protein of 55 kDa",
  "gene_symbol": "CEP55",
  "gene": "UniProtKB:Q53EZ4",
  "term_label": "establishment of protein localization",
  "term_id": "GO:0045184"
}